{
  "gene_symbol": "CHI3L1",
  "gene": "UniProtKB:P36222",
  "term_id": "UNKNOWN:0001",
  "term_label": "Unknown molecular function",
  "gene_name": "Chitinase-3-like protein 1"
}